{
  "gene_symbol": "MDGA1",
  "gene_name": "MAM domain-containing glycosylphosphatidylinositol anchor protein 1",
  "term_label": "Golgi apparatus",
  "term_id": "GO:0005794",
  "gene": "UniProtKB:Q8NFP4"
}